{
  "gene": "UniProtKB:P51686",
  "term_label": "calcium-mediated signaling",
  "gene_name": "C-C chemokine receptor type 9",
  "gene_symbol": "CCR9",
  "term_id": "GO:0019722"
}